taurocyamine kinase activity [GO:0050324] (molecular function) Sources: EC:2.7.3.4, RHEA:22516 Definition: Catalysis of the reaction: ATP + taurocyamine = N-phosphotaurocyamine + ADP + 2 H+. Relationships: is a type of GO:0016301; is a type of phosphotransferase activity, nitrogenous group as acceptor [GO:0016775] Also known as: ATP:taurocyamine N-phosphotransferase activity, ATP:taurocyamine phosphotransferase activity, taurocyamine phosphotransferase activity